{
  "gene_name": "Transmembrane protein 53",
  "term_id": "UNKNOWN:0002",
  "term_label": "Unknown biological process",
  "gene": "UniProtKB:Q6P2H8",
  "gene_symbol": "TMEM53"
}